{
  "gene_name": "UL16-binding protein 1",
  "gene": "UniProtKB:Q9BZM6",
  "term_label": "natural killer cell mediated cytotoxicity",
  "term_id": "GO:0042267",
  "gene_symbol": "ULBP1"
}